{
  "term_id": "GO:0016332",
  "gene": "UniProtKB:Q8N3R9",
  "term_label": "establishment or maintenance of polarity of embryonic epithelium",
  "gene_name": "Protein PALS1",
  "gene_symbol": "PALS1"
}